{
  "gene_symbol": "MON1A",
  "gene_name": "Vacuolar fusion protein MON1 homolog A",
  "term_label": "protein secretion",
  "term_id": "GO:0009306",
  "gene": "UniProtKB:Q86VX9"
}